diphosphoric monoester hydrolase activity [GO:0016794] (molecular function) Definition: Catalysis of the hydrolysis of a diphosphoester, releasing a diphosphate and a free hydroxyl group. Sources: EC:3.1.7.- Subtypes: guanosine-3',5'-bis(diphosphate) 3'-diphosphatase activity [GO:0008893], GO:0050210, (13E)-labda-7,13-dien-15-ol synthase activity [GO:0102305] Relationships: is a type of phosphoric ester hydrolase activity [GO:0042578]